D-proline reductase activity [GO:0050002] (molecular function) Also known as: 5-aminopentanoate:[PrdC protein] oxidoreductase (cyclizing) activity, D-proline reductase (dithiol) activity Definition: Catalysis of the reaction: 5-aminopentanoate + [PrdC protein]-Se-L-selenocysteinyl-S-L-cysteine = [PrdC protein]-L-selenocysteine/L-cysteine + D-proline. Sources: EC:1.21.4.1 Relationships: is a type of oxidoreductase activity, acting on X-H and Y-H to form an X-Y bond, with a disulfide as acceptor [GO:0050485]